ventricular cardiac muscle cell action potential [GO:0086005] (biological process) Relationships: is a type of cardiac muscle cell action potential involved in contraction [GO:0086002] Sources: GOC:BHF, GOC:mtg_cardiac_conduct_nov11 Regulation: RO_0002211 by regulation of ventricular cardiac muscle cell action potential [GO:0098911]; negatively regulated by negative regulation of ventricular cardiac muscle cell action potential [GO:1903946]; positively regulated by positive regulation of ventricular cardiac muscle cell action potential [GO:1903947] Definition: An action potential that occurs in a ventricular cardiac muscle cell.